cell projection morphogenesis [GO:0048858] (biological process) Sources: GO_REF:0000021 Subtypes: imaginal disc-derived wing hair outgrowth [GO:0035318], imaginal disc-derived wing hair elongation [GO:0035319], glial cell projection elongation [GO:0106091], plasma membrane bounded cell projection morphogenesis [GO:0120039] Definition: The process in which the anatomical structures of a cell projection are generated and organized. Relationships: is a type of GO:0009653; is a type of GO:0030030; is part of GO:0000902